{
  "gene": "UniProtKB:Q8WWF6",
  "term_label": "Unknown cellular component",
  "term_id": "UNKNOWN:0003",
  "gene_symbol": "DNAJB3",
  "gene_name": "DnaJ homolog subfamily B member 3"
}